protein localization to mating-type region heterochromatin [GO:1903212] (biological process) References: PMID:18761674 Sources: GOC:TermGenie, GO_REF:0000087 Definition: A process in which a protein is transported to, or maintained in, a location within a mating-type region heterochromatin. Also known as: protein localisation in mating-type region heterochromatin, protein localisation to mating-type region heterochromatin, protein localization in mating-type region heterochromatin Relationships: is a type of protein localization to heterochromatin [GO:0097355]